amphisome-lysosome fusion [GO:0061911] (biological process) References: PMID:24219988 Relationships: is_a vesicle fusion [GO:0006906]; is part of macroautophagy [GO:0016236] Definition: The process in which amphisomes fuse with a vacuole (yeast) or lysosome (e.g. mammals and insects). In the case of yeast, inner membrane-bounded structures (autophagic bodies) appear in the vacuole. Fusion provides an acidic environment and digestive function to the interior of the amphisome.